organellar voltage-gated chloride channel activity [GO:0015274] (molecular function) Relationships: is a type of voltage-gated chloride channel activity [GO:0005247] Sources: GOC:mtg_transport, ISBN:0815340729 Also known as: organellar voltage gated chloride channel activity, organellar voltage-dependent chloride channel activity Definition: Enables the transmembrane transfer of a chloride ion by a voltage-gated channel. The membrane is an organellar membrane.